{
  "term_label": "brain development",
  "gene_symbol": "CNTN1",
  "term_id": "GO:0007420",
  "gene_name": "Contactin-1",
  "gene": "UniProtKB:Q12860"
}